{
  "gene_symbol": "IGHV3-23",
  "term_id": "GO:0003823",
  "gene_name": "Immunoglobulin heavy variable 3-23",
  "term_label": "antigen binding",
  "gene": "UniProtKB:P01764"
}